{
  "gene_name": "Sialic acid-binding Ig-like lectin 5",
  "gene": "UniProtKB:O15389",
  "gene_symbol": "SIGLEC5",
  "term_label": "plasma membrane",
  "term_id": "GO:0005886"
}